{
  "gene_symbol": "OGDHL",
  "term_id": "GO:0006099",
  "term_label": "tricarboxylic acid cycle",
  "gene": "UniProtKB:Q9ULD0",
  "gene_name": "2-oxoglutarate dehydrogenase-like, mitochondrial"
}